{
  "term_label": "DNA binding",
  "term_id": "GO:0003677",
  "gene_name": "SOSS complex subunit B2",
  "gene": "UniProtKB:Q96AH0",
  "gene_symbol": "NABP1"
}